{
  "gene_name": "ETS-related transcription factor Elf-2",
  "gene": "UniProtKB:Q15723",
  "term_label": "cell differentiation",
  "term_id": "GO:0030154",
  "gene_symbol": "ELF2"
}